phosphagen biosynthetic process [GO:0042396] (biological process) Relationships: is a type of phosphate-containing compound metabolic process [GO:0006796]; is a type of GO:0042398; is_a organophosphate biosynthetic process [GO:0090407] Also known as: phosphagen anabolism, phosphagen biosynthesis, phosphagen formation, phosphagen synthesis Sources: GOC:jl, ISBN:0198506732 Definition: The chemical reactions and pathways resulting in the formation of phosphagen, any of a group of guanidine phosphates that occur in muscle and can be used to regenerate ATP from ADP during muscular contraction. Subtypes: phosphoarginine biosynthetic process [GO:0046312], phosphocreatine biosynthetic process [GO:0046314]